{
  "gene_name": "ATP synthase mitochondrial F1 complex assembly factor 1",
  "gene_symbol": "ATPAF1",
  "term_label": "mitochondrion",
  "gene": "UniProtKB:Q5TC12",
  "term_id": "GO:0005739"
}